{
  "gene_symbol": "SH3BP5",
  "gene_name": "SH3 domain-binding protein 5",
  "term_id": "GO:0005737",
  "gene": "UniProtKB:O60239",
  "term_label": "cytoplasm"
}